{
  "gene": "UniProtKB:O14810",
  "gene_symbol": "CPLX1",
  "term_id": "GO:0031201",
  "term_label": "SNARE complex",
  "gene_name": "Complexin-1"
}